{
  "term_id": "GO:0090575",
  "term_label": "RNA polymerase II transcription regulator complex",
  "gene_name": "Protein max",
  "gene": "UniProtKB:P61244",
  "gene_symbol": "MAX"
}